{
  "term_id": "UNKNOWN:0002",
  "term_label": "Unknown biological process",
  "gene_symbol": "GCAT",
  "gene": "UniProtKB:O75600",
  "gene_name": "2-amino-3-ketobutyrate coenzyme A ligase, mitochondrial"
}